{
  "term_label": "myosin filament",
  "gene_symbol": "MYH9",
  "term_id": "GO:0032982",
  "gene": "UniProtKB:P35579",
  "gene_name": "Myosin-9"
}